{
  "gene_symbol": "PRKAB1",
  "gene_name": "5'-AMP-activated protein kinase subunit beta-1",
  "gene": "UniProtKB:Q9Y478",
  "term_id": "GO:0005737",
  "term_label": "cytoplasm"
}